{
  "gene_symbol": "DNAJC5",
  "gene_name": "DnaJ homolog subfamily C member 5",
  "gene": "UniProtKB:Q9H3Z4",
  "term_label": "Unknown molecular function",
  "term_id": "UNKNOWN:0001"
}